{
  "term_id": "GO:0005634",
  "term_label": "nucleus",
  "gene": "UniProtKB:Q9H0K1",
  "gene_name": "Serine_threonine-protein kinase SIK2",
  "gene_symbol": "SIK2"
}